mesenchymal cell apoptotic process involved in metanephros development [GO:1900200] (biological process) Definition: Any mesenchymal cell apoptotic process that is involved in metanephros development. Also known as: mesenchymal cell apoptosis involved in metanephros development References: PMID:17314325 Sources: GOC:TermGenie, GOC:mtg_apoptosis, GOC:mtg_kidney_jan10, GOC:yaf Subtypes: mesenchymal cell apoptotic process involved in metanephric nephron morphogenesis [GO:1901147] Regulation: regulated by regulation of mesenchymal cell apoptotic process involved in metanephros development [GO:1900211]; negatively regulated by negative regulation of mesenchymal cell apoptotic process involved in metanephros development [GO:1900212]; positively regulated by positive regulation of mesenchymal cell apoptotic process involved in metanephros development [GO:1900213] Relationships: is a type of mesenchymal cell apoptotic process [GO:0097152]; is a type of GO:1902742; is part of metanephros development [GO:0001656]